{
  "term_id": "GO:0004748",
  "gene": "UniProtKB:Q7LG56",
  "gene_name": "Ribonucleoside-diphosphate reductase subunit M2 B",
  "gene_symbol": "RRM2B",
  "term_label": "ribonucleoside-diphosphate reductase activity, thioredoxin disulfide as acceptor"
}